{
  "gene_name": "Eukaryotic translation elongation factor 1 epsilon-1",
  "gene_symbol": "EEF1E1",
  "term_label": "Unknown biological process",
  "gene": "UniProtKB:O43324",
  "term_id": "UNKNOWN:0002"
}